{
  "term_id": "GO:0000139",
  "gene_symbol": "SLC35B2",
  "gene_name": "Adenosine 3'-phospho 5'-phosphosulfate transporter 1",
  "term_label": "Golgi membrane",
  "gene": "UniProtKB:Q8TB61"
}